{
  "gene_symbol": "CLDN19",
  "term_label": "apical junction assembly",
  "gene": "UniProtKB:Q8N6F1",
  "term_id": "GO:0043297",
  "gene_name": "Claudin-19"
}